regulation of fibroblast apoptotic process [GO:2000269] (biological process) Definition: Any process that modulates the frequency, rate or extent of fibroblast apoptotic process. Sources: GOC:mtg_apoptosis, GOC:obol, GOC:yaf Relationships: is a type of regulation of apoptotic process [GO:0042981]; regulates fibroblast apoptotic process [GO:0044346] Subtypes: negative regulation of fibroblast apoptotic process [GO:2000270], GO:2000271 Also known as: regulation of fibroblast apoptosis